{
  "gene": "UniProtKB:Q9NPA2",
  "term_label": "collagen catabolic process",
  "gene_symbol": "MMP25",
  "term_id": "GO:0030574",
  "gene_name": "Matrix metalloproteinase-25"
}